{
  "gene_symbol": "BAG1",
  "gene_name": "BAG family molecular chaperone regulator 1",
  "gene": "UniProtKB:Q99933",
  "term_label": "cytoplasm",
  "term_id": "GO:0005737"
}